{
  "term_label": "Unknown molecular function",
  "gene_name": "Neurotrimin",
  "gene": "UniProtKB:Q9P121",
  "gene_symbol": "NTM",
  "term_id": "UNKNOWN:0001"
}